{
  "gene": "UniProtKB:P46527",
  "term_label": "cytoplasm",
  "term_id": "GO:0005737",
  "gene_name": "Cyclin-dependent kinase inhibitor 1B",
  "gene_symbol": "CDKN1B"
}